{
  "gene_name": "V-set and immunoglobulin domain-containing protein 4",
  "gene": "UniProtKB:Q9Y279",
  "term_id": "GO:0032703",
  "term_label": "negative regulation of interleukin-2 production",
  "gene_symbol": "VSIG4"
}